{
  "gene_name": "cAMP-dependent protein kinase catalytic subunit gamma",
  "gene_symbol": "PRKACG",
  "gene": "UniProtKB:P22612",
  "term_label": "cAMP-dependent protein kinase activity",
  "term_id": "GO:0004691"
}